{
  "gene_symbol": "LNPK",
  "term_id": "GO:0071782",
  "gene_name": "Endoplasmic reticulum junction formation protein lunapark",
  "term_label": "endoplasmic reticulum tubular network",
  "gene": "UniProtKB:Q9C0E8"
}